{
  "term_label": "cell periphery",
  "gene_name": "Thrombospondin type-1 domain-containing protein 1",
  "gene": "UniProtKB:Q9NS62",
  "term_id": "GO:0071944",
  "gene_symbol": "THSD1"
}